{
  "gene_name": "Proton-coupled zinc antiporter SLC30A9, mitochondrial",
  "gene_symbol": "SLC30A9",
  "gene": "UniProtKB:Q6PML9",
  "term_label": "endoplasmic reticulum",
  "term_id": "GO:0005783"
}